mesenchymal stem cell migration involved in uteric bud morphogenesis [GO:0061456] (biological process) Relationships: is_a cell migration involved in kidney development [GO:0035787]; is part of ureteric bud morphogenesis [GO:0060675] Definition: The orderly movement of a mesenchymal stem cell from one site to another contributing to the shaping of the ureteric bud. A mesenchymal stem cell, or MSC, is a cell that retains the ability to divide and proliferate throughout life to provide progenitor cells that can differentiate into specialized mesenchymal cells. Sources: GOC:dph, GOC:tb